{
  "gene_symbol": "ZNF563",
  "gene_name": "Zinc finger protein 563",
  "term_label": "DNA-binding transcription factor activity, RNA polymerase II-specific",
  "gene": "UniProtKB:Q8TA94",
  "term_id": "GO:0000981"
}